{
  "term_id": "GO:1900029",
  "term_label": "positive regulation of ruffle assembly",
  "gene_symbol": "EPS8L1",
  "gene": "UniProtKB:Q8TE68",
  "gene_name": "Epidermal growth factor receptor kinase substrate 8-like protein 1"
}